{
  "term_id": "GO:0005665",
  "gene_symbol": "POLR2I",
  "gene": "UniProtKB:P36954",
  "term_label": "RNA polymerase II, core complex",
  "gene_name": "DNA-directed RNA polymerase II subunit RPB9"
}